regulation of Rho protein signal transduction [GO:0035023] (biological process) Definition: Any process that modulates the frequency, rate or extent of Rho protein signal transduction. Sources: GOC:bf Relationships: is a type of regulation of small GTPase mediated signal transduction [GO:0051056]; regulates Rho protein signal transduction [GO:0007266] Subtypes: regulation of Cdc42 protein signal transduction [GO:0032489], negative regulation of Rho protein signal transduction [GO:0035024], positive regulation of Rho protein signal transduction [GO:0035025]